{
  "term_id": "GO:0008307",
  "gene_name": "Myosin light chain 1_3, skeletal muscle isoform",
  "gene": "UniProtKB:P05976",
  "gene_symbol": "MYL1",
  "term_label": "structural constituent of muscle"
}